{
  "term_label": "actin crosslink formation",
  "gene_name": "Dihydropyrimidinase-related protein 3",
  "term_id": "GO:0051764",
  "gene": "UniProtKB:Q14195",
  "gene_symbol": "DPYSL3"
}